{
  "gene_name": "Immunoglobulin kappa variable 3-15",
  "gene_symbol": "IGKV3-15",
  "gene": "UniProtKB:P01624",
  "term_label": "immunoglobulin complex",
  "term_id": "GO:0019814"
}